{
  "gene": "UniProtKB:P05108",
  "gene_name": "Cholesterol side-chain cleavage enzyme, mitochondrial",
  "term_label": "cellular response to peptide hormone stimulus",
  "gene_symbol": "CYP11A1",
  "term_id": "GO:0071375"
}